{
  "term_id": "UNKNOWN:0002",
  "term_label": "Unknown biological process",
  "gene": "UniProtKB:P29508",
  "gene_symbol": "SERPINB3",
  "gene_name": "Serpin B3"
}